rod photoreceptor disc lumen [GO:0120203] (cellular component) Definition: The volume enclosed by the membrane of a rod photoreceptor cell disc membrane. References: PMID:19501669, PMID:26574505, PMID:6771304 Sources: GOC:krc, GOC:pde Relationships: is_a GO:0043233; is part of GO:0120200